cytoplasm to vacuole targeting by the NVT pathway [GO:0120113] (biological process) Definition: A pathway targeting soluble cytosolic proteins to the vacuole lumen. It uses a selective autophagy receptor protein Nbr1, which is an ortholog of mammalian NBR1, and is remotely related to S. cerevisiae Cvt pathway receptor protein Atg19. Similar to the Cvt pathway, the cargos transported by this pathway are hydrolases, which presumably contribute to the hydrolytic activities in the vacuole lumen. Different from the Cvt pathway, this pathway does not require the macroautophagy machinery, but instead relies on the ESCRT machinery for cargo sequestration. This pathway is observed in the fission yeast S. pombe. References: PMID:26365378 Also known as: protein localization by the Nbr1-mediated vacuolar targeting pathway Relationships: is a type of protein targeting to vacuole [GO:0006623]; has part vacuolar protein processing [GO:0006624]